{
  "gene": "UniProtKB:P01704",
  "gene_name": "Immunoglobulin lambda variable 2-14",
  "gene_symbol": "IGLV2-14",
  "term_label": "Unknown molecular function",
  "term_id": "UNKNOWN:0001"
}